{
  "gene_symbol": "PSMC3IP",
  "gene": "UniProtKB:Q9P2W1",
  "gene_name": "Homologous-pairing protein 2 homolog",
  "term_label": "condensed nuclear chromosome",
  "term_id": "GO:0000794"
}